{
  "term_id": "UNKNOWN:0003",
  "gene_name": "Uncharacterized protein C13orf42",
  "gene_symbol": "C13orf42",
  "gene": "UniProtKB:A0A1B0GVH6",
  "term_label": "Unknown cellular component"
}